mycophenolic acid biosynthetic process [GO:0140722] (biological process) References: PMID:21398490, PMID:26751579, PMID:31209052 Definition: The chemical reactions and pathways resulting in the formation of mycophenolic acid (MPA). MPA is the first isolated antibiotic natural product in the world obtained from a culture of Penicillium brevicompactum in 1893. Relationships: is a type of antibiotic biosynthetic process [GO:0017000]; is a type of polyketide biosynthetic process [GO:0030639]; is a type of GO:0043386; is_a phenol-containing compound biosynthetic process [GO:0046189]; is a type of monocarboxylic acid biosynthetic process [GO:0072330]; is a type of lactone biosynthetic process [GO:1901336] Also known as: MPA anabolism, MPA biosynthesis, MPA formation, MPA synthesis, mycophenolic acid anabolism, mycophenolic acid biosynthesis, mycophenolic acid formation, mycophenolic acid synthesis